S-succinylglutathione hydrolase activity [GO:0050273] (molecular function) Definition: Catalysis of the reaction: S-succinylglutathione + H2O = glutathione + H+ + succinate. Sources: EC:3.1.2.13, RHEA:16713 Relationships: is a type of thiolester hydrolase activity [GO:0016790]